{
  "term_id": "GO:0046655",
  "gene": "UniProtKB:P00374",
  "gene_symbol": "DHFR",
  "gene_name": "Dihydrofolate reductase",
  "term_label": "folic acid metabolic process"
}